{
  "term_id": "UNKNOWN:0002",
  "gene_name": "Keratin-associated protein 3-3",
  "gene_symbol": "KRTAP3-3",
  "term_label": "Unknown biological process",
  "gene": "UniProtKB:Q9BYR6"
}